{
  "gene_name": "ADP_ATP translocase 2",
  "gene": "UniProtKB:P05141",
  "term_id": "GO:0005743",
  "gene_symbol": "SLC25A5",
  "term_label": "mitochondrial inner membrane"
}